{
  "term_label": "heteromeric SMAD protein complex",
  "gene_name": "Mothers against decapentaplegic homolog 3",
  "term_id": "GO:0071144",
  "gene_symbol": "SMAD3",
  "gene": "UniProtKB:P84022"
}